{
  "gene": "UniProtKB:Q6ZN03",
  "gene_name": "Putative uncharacterized protein encoded by LINC00322",
  "term_id": "UNKNOWN:0001",
  "term_label": "Unknown molecular function",
  "gene_symbol": "LINC00322"
}